{
  "term_id": "GO:0003924",
  "term_label": "GTPase activity",
  "gene_symbol": "RIT1",
  "gene": "UniProtKB:Q92963",
  "gene_name": "GTP-binding protein Rit1"
}